{
  "gene_symbol": "BMF",
  "gene_name": "Bcl-2-modifying factor",
  "term_id": "GO:0016459",
  "gene": "UniProtKB:Q96LC9",
  "term_label": "myosin complex"
}